leaf senescence [GO:0010150] (biological process) References: PMID:17177638, PMID:34938309 Sources: ISBN:0387987819 Regulation: RO_0002211 by GO:1900055; negatively regulated by GO:1900056; positively regulated by positive regulation of leaf senescence [GO:1900057] Relationships: is a type of GO:0090693; is part of GO:0048366 Definition: The last stage of leaf development during which programmed degradation of macromolecules and nutrient recycling take place.